{
  "gene_name": "Beta-galactoside alpha-2,6-sialyltransferase 2",
  "gene_symbol": "ST6GAL2",
  "term_id": "GO:0003835",
  "term_label": "beta-galactoside alpha-2,6-sialyltransferase activity",
  "gene": "UniProtKB:Q96JF0"
}